metanephric tubule development [GO:0072170] (biological process) Definition: The progression of a metanephric tubule over time, from its initial formation to the mature structure. A metanephric tubule is an epithelial tube that is part of the metanephros. Subtypes: metanephric nephron tubule development [GO:0072234] Relationships: is a type of tube development [GO:0035295]; is a type of metanephric epithelium development [GO:0072207] Sources: GOC:mtg_kidney_jan10